{
  "gene_symbol": "ADARB2",
  "term_id": "GO:0008251",
  "gene_name": "Double-stranded RNA-specific editase B2",
  "term_label": "tRNA-specific adenosine deaminase activity",
  "gene": "UniProtKB:Q9NS39"
}